negative regulation of transformation of host cell by virus [GO:1904188] (biological process) Also known as: down regulation of transformation of host cell by virus, down regulation of viral transformation, down regulation of viral transformation of host cell, down-regulation of transformation of host cell by virus, down-regulation of viral transformation, down-regulation of viral transformation of host cell, downregulation of transformation of host cell by virus, downregulation of viral transformation, downregulation of viral transformation of host cell, negative regulation of viral transformation, negative regulation of viral transformation of host cell, inhibition of transformation of host cell by virus, inhibition of viral transformation, inhibition of viral transformation of host cell Relationships: is a type of GO:0048519; is a type of regulation of transformation of host cell by virus [GO:1904187]; negatively regulates symbiont-mediated transformation of host cell [GO:0019087] Definition: Any process that stops, prevents or reduces the frequency, rate or extent of transformation of host cell by virus. References: PMID:12200142 Sources: GOC:TermGenie, GO_REF:0000058